RNA glycosylase activity [GO:0030597] (molecular function) Definition: Catalysis of the hydrolysis of N-glycosidic bonds in an RNA molecule. Subtypes: rRNA N-glycosylase activity [GO:0030598] Sources: GOC:mah Relationships: is a type of hydrolase activity, hydrolyzing N-glycosyl compounds [GO:0016799]; is a type of catalytic activity, acting on RNA [GO:0140098]